{
  "gene": "UniProtKB:Q9BYQ7",
  "term_id": "UNKNOWN:0001",
  "gene_name": "Keratin-associated protein 4-1",
  "term_label": "Unknown molecular function",
  "gene_symbol": "KRTAP4-1"
}